phenanthrene catabolic process via trans-9(S),10(S)-dihydrodiolphenanthrene [GO:0018957] (biological process) Definition: The chemical reactions and pathways resulting in the breakdown of phenanthrene, a tricyclic aromatic hydrocarbon, where trans-9(S),10(S)-dihydrodiolphenanthrene is the principal intermediate metabolite. Also known as: phenanthrene breakdown via trans-9(S),10(S)-dihydrodiolphenanthrene, phenanthrene degradation via trans-9(S),10(S)-dihydrodiolphenanthrene Relationships: is a type of GO:0042216 Sources: UM-BBD_pathwayID:pha2